{
  "gene_symbol": "MAP3K6",
  "gene_name": "Mitogen-activated protein kinase kinase kinase 6",
  "term_id": "UNKNOWN:0003",
  "gene": "UniProtKB:O95382",
  "term_label": "Unknown cellular component"
}